{
  "gene_name": "RING finger protein 150",
  "gene": "UniProtKB:Q9ULK6",
  "term_id": "GO:0061630",
  "term_label": "ubiquitin protein ligase activity",
  "gene_symbol": "RNF150"
}